medium-chain fatty acid biosynthetic process [GO:0051792] (biological process) Note: While there is not universal consensus on the lengths of short-, medium-, long- and very-long-chain fatty acids, the GO uses the definitions in ChEBI (see CHEBI:26666, CHEBI:59554, CHEBI:15904 and CHEBI:27283). Also known as: medium chain fatty acid biosynthesis, medium chain fatty acid biosynthetic process, medium-chain fatty acid anabolism, medium-chain fatty acid biosynthesis, medium-chain fatty acid formation, medium-chain fatty acid synthesis Sources: Wikipedia:Fatty_acid_metabolism Definition: The chemical reactions and pathways resulting in the formation of a medium-chain fatty acid. A medium-chain fatty acid has an aliphatic tail containing 6 to 12 carbons. Relationships: is a type of fatty acid biosynthetic process [GO:0006633]; is a type of medium-chain fatty acid metabolic process [GO:0051791]